{
  "term_label": "IgG binding",
  "gene": "UniProtKB:P31995",
  "term_id": "GO:0019864",
  "gene_symbol": "FCGR2C",
  "gene_name": "Low affinity immunoglobulin gamma Fc region receptor II-c"
}